{
  "gene": "UniProtKB:Q8TCH9",
  "gene_name": "Putative uncharacterized protein FLJ23865",
  "term_id": "UNKNOWN:0003",
  "term_label": "Unknown cellular component",
  "gene_symbol": "Q8TCH9"
}